{
  "gene": "UniProtKB:O75897",
  "term_id": "GO:0004062",
  "gene_symbol": "SULT1C4",
  "gene_name": "Sulfotransferase 1C4",
  "term_label": "aryl sulfotransferase activity"
}